{
  "term_id": "GO:0006357",
  "term_label": "regulation of transcription by RNA polymerase II",
  "gene_name": "NK1 transcription factor-related protein 1",
  "gene_symbol": "NKX1-1",
  "gene": "UniProtKB:Q15270"
}